{
  "gene": "UniProtKB:Q9Y2K3",
  "gene_name": "Myosin-15",
  "term_id": "GO:0000146",
  "gene_symbol": "MYH15",
  "term_label": "microfilament motor activity"
}